mammary gland lobule development [GO:0061377] (biological process) Definition: The progression of the mammary gland lobule over time, from its formation to the mature structure. A mammary gland lobule is a small rounded projection of the mammary gland. Relationships: is_a GO:0048856; is part of mammary gland development [GO:0030879] Sources: GOC:dph, GOC:yaf